ubiquitin-protein transferase activator activity [GO:0097027] (molecular function) Definition: Binds to and increases the activity of a ubiquitin-protein transferase. References: PMID:18321851 Sources: GOC:rb Relationships: is a type of GO:0008047; is a type of ubiquitin-protein transferase regulator activity [GO:0055106]; positively regulates ubiquitin-protein transferase activity [GO:0004842] Subtypes: ubiquitin ligase activator activity [GO:1990757]